{
  "term_label": "early endosome",
  "gene_symbol": "RAB20",
  "gene": "UniProtKB:Q9NX57",
  "term_id": "GO:0005769",
  "gene_name": "Ras-related protein Rab-20"
}